{
  "term_label": "neuron differentiation",
  "gene": "UniProtKB:O00570",
  "gene_symbol": "SOX1",
  "gene_name": "Transcription factor SOX-1",
  "term_id": "GO:0030182"
}